{
  "term_id": "GO:0007155",
  "gene_name": "Tyrosine-protein kinase Fes_Fps",
  "gene_symbol": "FES",
  "gene": "UniProtKB:P07332",
  "term_label": "cell adhesion"
}